{
  "term_label": "late endosome",
  "gene": "UniProtKB:P51151",
  "gene_symbol": "RAB9A",
  "gene_name": "Ras-related protein Rab-9A",
  "term_id": "GO:0005770"
}